apicomplexan dense granule membrane [GO:0030668] (cellular component) Definition: The lipid bilayer surrounding a dense granule of the type found in apicomplexan parasites. Relationships: is a type of secretory granule membrane [GO:0030667]; is part of apicomplexan dense granule [GO:0020026] Sources: GOC:mah, GOC:mtg_sensu